bacterial extracellular vesicle [GO:0097691] (cellular component) Definition: Small membrane vesicle (< 1 um) that buds off a prokaryotic cell plasma membrane, able to carry proteins, phospholipids, lipopolysaccharides, nucleic acids, viruses, and more. Important in intercellular communication and pathogenesis; can exist within host cells. Relationships: is a type of extracellular vesicle [GO:1903561] References: PMID:25704309 Sources: GOC:aa